{
  "term_id": "GO:0003676",
  "gene_name": "Shadow of prion protein",
  "term_label": "nucleic acid binding",
  "gene_symbol": "SPRN",
  "gene": "UniProtKB:Q5BIV9"
}